{
  "term_label": "Unknown biological process",
  "gene_symbol": "ARMC12",
  "gene_name": "Armadillo repeat-containing protein 12",
  "term_id": "UNKNOWN:0002",
  "gene": "UniProtKB:Q5T9G4"
}